positive regulation of formation of structure involved in a symbiotic process [GO:0044149] (biological process) Definition: Any process that activates or increases the frequency, rate or extent of the progression of an organism from an initial condition to a later condition, occurring in, on or near the exterior of its host organism. Relationships: is a type of GO:0044145; is a type of positive regulation of biological process [GO:0048518]; positively regulates formation of structure involved in a symbiotic process [GO:0044111] Subtypes: GO:0044129, positive regulation of formation by symbiont of haustorium for nutrient acquisition from host [GO:0075046], positive regulation of arbuscule formation for nutrient acquisition from host [GO:0075330] Also known as: positive regulation of development of symbiont during interaction with host, positive regulation of development of symbiont involved in interaction with host Note: This term partially replaces the obsolete term 'positive regulation of growth or development of symbiont during interaction with host ; GO:0075339'. See also 'positive regulation of growth of symbiont during interaction with host ; GO:0044148'. Sources: GOC:jl, GOC:pamgo_curators